{
  "gene_name": "Putative small nuclear ribonucleoprotein G-like protein 15",
  "term_label": "U4 snRNP",
  "term_id": "GO:0005687",
  "gene_symbol": "SNRPGP15",
  "gene": "UniProtKB:A8MWD9"
}